insulin control element activator complex [GO:0030232] (cellular component) References: PMID:7935390 Definition: Transcription factor complex that binds to the insulin control element (ICE), a DNA sequence element found within the 5'-flanking region of the insulin gene, and activates ICE-mediated transcription. Also known as: ICE activator complex Relationships: is a type of RNA polymerase II transcription regulator complex [GO:0090575]